phosphatidyl-N-monomethylethanolamine biosynthetic process [GO:0006647] (biological process) Definition: The chemical reactions and pathways involving phosphatidyl-N-monomethylethanolamine (PMME), a derivative of phosphatidylethanolamine with a methylated amine group. Also known as: PMME biosynthesis, PMME biosynthetic process, phosphatidyl-N-monomethylethanolamine anabolism, phosphatidyl-N-monomethylethanolamine biosynthesis, phosphatidyl-N-monomethylethanolamine formation, phosphatidyl-N-monomethylethanolamine synthesis Relationships: is a type of phosphatidylethanolamine biosynthetic process [GO:0006646] References: PMID:35071223